{
  "gene_symbol": "CDK17",
  "gene": "UniProtKB:Q00537",
  "term_label": "cyclin-dependent protein serine/threonine kinase activity",
  "gene_name": "Cyclin-dependent kinase 17",
  "term_id": "GO:0004693"
}